{
  "term_label": "cytoplasm",
  "gene_symbol": "KHK",
  "gene_name": "Ketohexokinase",
  "term_id": "GO:0005737",
  "gene": "UniProtKB:P50053"
}